{
  "gene": "UniProtKB:Q13118",
  "gene_symbol": "KLF10",
  "term_label": "regulation of transcription by RNA polymerase II",
  "gene_name": "Krueppel-like factor 10",
  "term_id": "GO:0006357"
}